{
  "gene_symbol": "CPNE7",
  "term_label": "cellular response to calcium ion",
  "gene_name": "Copine-7",
  "gene": "UniProtKB:Q9UBL6",
  "term_id": "GO:0071277"
}